{
  "term_label": "cysteine-type endopeptidase inhibitor activity involved in apoptotic process",
  "gene_name": "Baculoviral IAP repeat-containing protein 2",
  "gene_symbol": "BIRC2",
  "term_id": "GO:0043027",
  "gene": "UniProtKB:Q13490"
}